stretch-activated, monoatomic cation-selective, calcium channel activity involved in regulation of action potential [GO:0097364] (molecular function) Relationships: is a type of stretch-activated, monoatomic cation-selective, calcium channel activity [GO:0015275]; regulates action potential [GO:0001508] Definition: Enables the transmembrane transfer of a calcium ion by a channel that opens in response to a mechanical stress in the form of stretching, and contributing to the regulation of action potential. Subtypes: stretch-activated, monoatomic cation-selective, calcium channel activity involved in regulation of cardiac muscle cell action potential [GO:0097365] References: PMID:21290758 Sources: GOC:BHF, GOC:mtg_cardiac_conduct_nov11 Also known as: stretch-activated, cation-selective, calcium channel activity involved in regulation of action potential